{
  "gene_symbol": "GRIN1",
  "term_label": "ionotropic glutamate receptor signaling pathway",
  "gene_name": "Glutamate receptor ionotropic, NMDA 1",
  "gene": "UniProtKB:Q05586",
  "term_id": "GO:0035235"
}